{
  "gene_symbol": "EPHA3",
  "term_id": "GO:0005005",
  "gene_name": "Ephrin type-A receptor 3",
  "term_label": "transmembrane-ephrin receptor activity",
  "gene": "UniProtKB:P29320"
}